propionate-CoA ligase activity [GO:0050218] (molecular function) Relationships: is a type of short-chain fatty acid-CoA ligase activity [GO:0031955] Definition: Catalysis of the reaction: ATP + propanoate + CoA = AMP + diphosphate + propanoyl-CoA. Also known as: propanoate:CoA ligase (AMP-forming), propionyl-CoA synthetase activity Sources: EC:6.2.1.17, MetaCyc:PROPIONATE--COA-LIGASE-RXN